{
  "term_label": "galactosylgalactosylxylosylprotein 3-beta-glucuronosyltransferase activity",
  "gene_name": "Galactosylgalactosylxylosylprotein 3-beta-glucuronosyltransferase 2",
  "term_id": "GO:0015018",
  "gene_symbol": "B3GAT2",
  "gene": "UniProtKB:Q9NPZ5"
}